positive regulation of protein ubiquitination [GO:0031398] (biological process) Also known as: up regulation of protein ubiquitination, up-regulation of protein ubiquitination, upregulation of protein ubiquitination, activation of protein ubiquitination, stimulation of protein ubiquitination Subtypes: positive regulation of ubiquitin-protein transferase activity [GO:0051443], positive regulation of protein autoubiquitination [GO:1902499], GO:1902527, positive regulation of protein polyubiquitination [GO:1902916] Definition: Any process that activates or increases the frequency, rate or extent of the addition of ubiquitin groups to a protein. Sources: GOC:mah Relationships: is a type of GO:0031396; is_a GO:1903322; positively regulates protein ubiquitination [GO:0016567]